{
  "gene": "UniProtKB:Q9UKI2",
  "term_label": "Rho protein signal transduction",
  "term_id": "GO:0007266",
  "gene_symbol": "CDC42EP3",
  "gene_name": "Cdc42 effector protein 3"
}